RNA decapping complex [GO:0098745] (cellular component) References: PMID:22323607 Sources: GOC:dos, GOC:vw Also known as: Dcp1-Dcp2 complex Definition: A protein complex consisting of a Dcp1 regulatory subunit and a Dcp2 catalytic subunit that has mRNA cap binding activity and is involved in decapping of nuclear-transcribed mRNA. Relationships: is a type of protein-containing complex [GO:0032991] Note: Additional components may be present, for example in ascomycetes this complex includes an additional regulatory subunit, Edc1.